{
  "gene_name": "WD repeat domain phosphoinositide-interacting protein 1",
  "term_id": "GO:0032266",
  "gene_symbol": "WIPI1",
  "gene": "UniProtKB:Q5MNZ9",
  "term_label": "phosphatidylinositol-3-phosphate binding"
}